{
  "term_label": "DNA-binding transcription factor activity, RNA polymerase II-specific",
  "gene_symbol": "ETV3L",
  "term_id": "GO:0000981",
  "gene_name": "ETS translocation variant 3-like protein",
  "gene": "UniProtKB:Q6ZN32"
}